{
  "term_label": "cytoplasmic cyclin-dependent protein kinase holoenzyme complex",
  "gene_name": "Cyclin-Y",
  "gene": "UniProtKB:Q8ND76",
  "gene_symbol": "CCNY",
  "term_id": "GO:0000308"
}